sphingoid long-chain base transport [GO:1905329] (biological process) Definition: The directed movement of a sphingoid long-chain base, sometimes referred to as long-chain base, or sphingoid base, into, out of or within a cell, or between cells, by means of some agent such as a transporter or pore. Sphingoid long-chain bases are long-chain aliphatic amines that are the fundamental building blocks of sphingolipids. The main mammalian sphingoid long-chain bases are dihydrosphingosine and sphingosine, while dihydrosphingosine and phytosphingosine are the main sphingoid long-chain bases in yeast. Relationships: is a type of GO:0006869; is a type of organic cation transport [GO:0015695]; is a type of nitrogen compound transport [GO:0071705] References: PMID:27136724 Sources: GOC:TermGenie, GOC:rn, GO_REF:0000065 Also known as: sphingoid base(1+) transport, dihydrosphingosine transport, phytosphingosine transport, sphingosine transport, long-chain base transport, sphingoid transport